peptidyl-tyrosine dephosphorylation involved in inactivation of protein kinase activity [GO:1990264] (biological process) Definition: Any peptidyl-tyrosine dephosphorylation that is involved in inactivation of protein kinase activity. References: PMID:7501024 Relationships: is a type of peptidyl-tyrosine dephosphorylation [GO:0035335]; BFO_0000050 negative regulation of protein kinase activity [GO:0006469]